{
  "term_id": "GO:0005737",
  "gene_symbol": "HOMER3",
  "term_label": "cytoplasm",
  "gene_name": "Homer protein homolog 3",
  "gene": "UniProtKB:Q9NSC5"
}